purine-containing compound biosynthetic process [GO:0072522] (BP) Relationships: is a type of GO:0009058; is_a purine-containing compound metabolic process [GO:0072521] Also known as: purine and derivative biosynthetic process, purine-containing compound anabolism, purine-containing compound biosynthesis, purine-containing compound formation, purine-containing compound synthesis Subtypes: purine nucleotide biosynthetic process [GO:0006164], GO:0009113, purine alkaloid biosynthetic process [GO:0009711], coenzyme A biosynthetic process [GO:0015937], zeatin biosynthetic process [GO:0033398], GO:0034033, isopentenyl adenine biosynthetic process [GO:0034265], discadenine biosynthetic process [GO:0034268], GO:0034418, purine nucleoside biosynthetic process [GO:0042451], purine-containing compound salvage [GO:0043101], acyl-CoA biosynthetic process [GO:0071616] Definition: The chemical reactions and pathways resulting in the formation of a purine-containing compound, i.e. any compound that contains purine or a formal derivative thereof. Sources: GOC:mah